dihydroneopterin monophosphate phosphatase activity [GO:0019176] (molecular function) Definition: Catalysis of the reaction: dihydroneopterin monophosphate = dihydroneopterin + phosphate. Sources: MetaCyc:DIHYDRONEOPTERIN-MONO-P-DEPHOS-RXN Also known as: dihydroneopterin monophosphate dephosphorylase activity Relationships: is a type of hydrolase activity, acting on acid anhydrides, in phosphorus-containing anhydrides [GO:0016818]